daunorubicin metabolic process [GO:0044597] (biological process) Definition: The chemical reactions and pathways involving daunorubicin, a chemotherapeutic of the anthracycline family that is given as a treatment for some types of cancer. Subtypes: GO:1901770, daunorubicin biosynthetic process [GO:1901771] Relationships: is a type of GO:0016137; is a type of polyketide metabolic process [GO:0030638]; is a type of ketone metabolic process [GO:0042180] References: PMID:20837989